{
  "gene": "UniProtKB:P55017",
  "gene_name": "Solute carrier family 12 member 3",
  "gene_symbol": "SLC12A3",
  "term_label": "apical plasma membrane",
  "term_id": "GO:0016324"
}